negative regulation of receptor-mediated endocytosis involved in cholesterol transport [GO:1905601] (BP) Definition: Any process that stops, prevents or reduces the frequency, rate or extent of receptor-mediated endocytosis involved in cholesterol transport. Relationships: is a type of GO:0032384; is a type of GO:0048261; is a type of regulation of receptor-mediated endocytosis involved in cholesterol transport [GO:1905600]; negatively regulates GO:0090118 Also known as: down regulation of receptor-mediated endocytosis involved in cholesterol transport, down-regulation of receptor-mediated endocytosis involved in cholesterol transport, downregulation of receptor-mediated endocytosis involved in cholesterol transport, inhibition of receptor-mediated endocytosis involved in cholesterol transport, inhibition of receptor-mediated endocytosis of LDL, down regulation of receptor-mediated endocytosis involved in intracellular cholesterol transport, down regulation of receptor-mediated endocytosis of LDL, down regulation of receptor-mediated endocytosis of low-density lipoprotein involved in cholesterol transport, down regulation of receptor-mediated endocytosis of low-density lipoprotein particle involved in cholesterol transport, down-regulation of receptor-mediated endocytosis involved in intracellular cholesterol transport, down-regulation of receptor-mediated endocytosis of LDL, down-regulation of receptor-mediated endocytosis of low-density lipoprotein involved in cholesterol transport, down-regulation of receptor-mediated endocytosis of low-density lipoprotein particle involved in cholesterol transport, downregulation of receptor-mediated endocytosis involved in intracellular cholesterol transport, downregulation of receptor-mediated endocytosis of LDL, downregulation of receptor-mediated endocytosis of low-density lipoprotein involved in cholesterol transport, downregulation of receptor-mediated endocytosis of low-density lipoprotein particle involved in cholesterol transport, inhibition of receptor-mediated endocytosis involved in intracellular cholesterol transport, inhibition of receptor-mediated endocytosis of low-density lipoprotein involved in cholesterol transport, inhibition of receptor-mediated endocytosis of low-density lipoprotein particle involved in cholesterol transport, negative regulation of receptor-mediated endocytosis involved in intracellular cholesterol transport, negative regulation of receptor-mediated endocytosis of LDL, negative regulation of receptor-mediated endocytosis of low-density lipoprotein involved in cholesterol transport, negative regulation of receptor-mediated endocytosis of low-density lipoprotein particle involved in cholesterol transport References: PMID:22848640 Sources: GOC:BHF, GOC:TermGenie, GOC:nc, GO_REF:0000058